{
  "gene_symbol": "OMP",
  "gene": "UniProtKB:P47874",
  "term_label": "axon",
  "gene_name": "Olfactory marker protein",
  "term_id": "GO:0030424"
}